{
  "term_label": "amino acid transport",
  "gene_symbol": "SLC6A16",
  "gene": "UniProtKB:Q9GZN6",
  "gene_name": "Orphan sodium- and chloride-dependent neurotransmitter transporter NTT5",
  "term_id": "GO:0006865"
}